{
  "term_label": "Unknown biological process",
  "term_id": "UNKNOWN:0002",
  "gene_name": "PiggyBac transposable element-derived protein 2",
  "gene_symbol": "PGBD2",
  "gene": "UniProtKB:Q6P3X8"
}